NADPH dehydrogenase activity [GO:0003959] (molecular function) Definition: Catalysis of the reaction: NADPH + H+ + acceptor = NADP+ + reduced acceptor. Sources: RHEA:13149 Also known as: NADPH diaphorase activity, NADPH-dehydrogenase activity, NADPH2 diaphorase activity, NADPH2-dehydrogenase activity, NADPH:(acceptor) oxidoreductase activity, NADPH:acceptor oxidoreductase activity, OYE, TPNH dehydrogenase activity, TPNH-diaphorase activity, dihydronicotinamide adenine dinucleotide phosphate dehydrogenase activity, old yellow enzyme, reduced nicotinamide adenine dinucleotide phosphate dehydrogenase activity, triphosphopyridine diaphorase activity, triphosphopyridine nucleotide diaphorase activity Relationships: is a type of oxidoreductase activity, acting on NAD(P)H [GO:0016651] Subtypes: quinone reductase (NADPH) activity [GO:0003960], NADPH dehydrogenase (quinone) activity [GO:0008753]